ureide biosynthetic process [GO:0010137] (biological process) Also known as: ureide anabolism, ureide biosynthesis, ureide formation, ureide synthesis Definition: The chemical reactions and pathways resulting in the formation of ureide, the organic form of nitrogen in nitrogen fixing and transporting plants, from IMP, which is synthesized de novo during nitrogen fixation by roots. Sources: GOC:pz Relationships: is a type of amide biosynthetic process [GO:0043604]